regulation of complement activation, lectin pathway [GO:0001868] (biological process) Definition: Any process that modulates the frequency, rate or extent of the lectin pathway of complement activation. Subtypes: GO:0001869, positive regulation of complement activation, lectin pathway [GO:0001870] Also known as: regulation of complement cascade, lectin pathway Sources: GOC:add, ISBN:0781735149 Relationships: is_a regulation of complement activation [GO:0030449]; is a type of regulation of innate immune response [GO:0045088]; regulates complement activation, lectin pathway [GO:0001867]